positive regulation of mRNA metabolic process [GO:1903313] (biological process) Definition: Any process that activates or increases the frequency, rate or extent of mRNA metabolic process. Sources: GOC:TermGenie, GOC:vw, GO_REF:0000058 Also known as: positive regulation of mRNA metabolism, up regulation of mRNA metabolic process, up regulation of mRNA metabolism, up-regulation of mRNA metabolic process, up-regulation of mRNA metabolism, upregulation of mRNA metabolic process, upregulation of mRNA metabolism, activation of mRNA metabolic process, activation of mRNA metabolism Relationships: is a type of positive regulation of RNA metabolic process [GO:0051254]; is a type of regulation of mRNA metabolic process [GO:1903311]; positively regulates mRNA metabolic process [GO:0016071] Subtypes: positive regulation of mRNA processing [GO:0050685], positive regulation of mRNA catabolic process [GO:0061014], positive regulation of mRNA modification [GO:0090366]